{
  "gene_name": "Caveolae-associated protein 3",
  "gene": "UniProtKB:Q969G5",
  "term_label": "Unknown biological process",
  "gene_symbol": "CAVIN3",
  "term_id": "UNKNOWN:0002"
}